{
  "gene_name": "Protein SDA1 homolog",
  "term_id": "GO:0042273",
  "gene_symbol": "SDAD1",
  "gene": "UniProtKB:Q9NVU7",
  "term_label": "ribosomal large subunit biogenesis"
}